arachidonate omega-hydroxylase activity [GO:0052869] (molecular function) Also known as: arachidonic acid hydroxylase activity, arachidonic acid omega-hydroxylase activity, arachidonic acid:oxygen 1-oxidoreductase activity Relationships: is a type of oxidoreductase activity, acting on paired donors, with incorporation or reduction of molecular oxygen, reduced flavin or flavoprotein as one donor, and incorporation of one atom of oxygen [GO:0016712] Sources: RHEA:39755 Definition: Catalysis of the reaction: (5Z,8Z,11Z,14Z)-eicosatetraenoate + O2 + reduced [NADPH--hemoprotein reductase] = 20-hydroxy-(5Z,8Z,11Z,14Z)-eicosatetraenoate + H+ + H2O + oxidized [NADPH--hemoprotein reductase]. (5Z,8Z,11Z,14Z)-icosatetraenoic acid is also known as arachidonic acid is also and 20-hydroxy-(5Z,8Z,11Z,14Z)-eicosatetraenoate as 20-HETE.